urea import across plasma membrane [GO:0140201] (biological process) References: PMID:17218313 Definition: The directed movement of urea from outside of a cell, across the plasma membrane and into the cytosol. Relationships: is a type of urea transmembrane transport [GO:0071918]; is a type of GO:0098739